hemoglobin catabolic process [GO:0042540] (biological process) Note: Note that 'hydrolysis' is actually a reaction rather than a process. The synonym 'hemoglobin hydrolysis' was the text string associated with the secondary ID GO:0020029, which was retained because its definition did describe a process. Also known as: haemoglobin catabolic process, haemoglobin catabolism, hemoglobin breakdown, hemoglobin catabolism, hemoglobin degradation, haemoglobin hydrolysis, hemoglobin hydrolysis Definition: The chemical reactions and pathways resulting in the breakdown of hemoglobin, an oxygen carrying, conjugated protein containing four heme groups and globin; especially, the proteolytic cleavage of hemoglobin to yield free heme, peptides, and amino acids. Sources: GOC:jl, GOC:mb Relationships: is_a hemoglobin metabolic process [GO:0020027]; is a type of protein catabolic process [GO:0030163]